{
  "term_id": "GO:0008330",
  "term_label": "protein tyrosine/threonine phosphatase activity",
  "gene": "UniProtKB:Q16829",
  "gene_name": "Dual specificity protein phosphatase 7",
  "gene_symbol": "DUSP7"
}